{
  "term_label": "Unknown molecular function",
  "term_id": "UNKNOWN:0001",
  "gene_symbol": "LYSMD2",
  "gene": "UniProtKB:Q8IV50",
  "gene_name": "LysM and putative peptidoglycan-binding domain-containing protein 2"
}